{
  "gene_symbol": "HES3",
  "term_id": "GO:0000981",
  "term_label": "DNA-binding transcription factor activity, RNA polymerase II-specific",
  "gene_name": "Transcription factor HES-3",
  "gene": "UniProtKB:Q5TGS1"
}